{
  "term_id": "GO:0004175",
  "gene_symbol": "PSMB5",
  "term_label": "endopeptidase activity",
  "gene": "UniProtKB:P28074",
  "gene_name": "Proteasome subunit beta type-5"
}